{
  "term_id": "UNKNOWN:0002",
  "gene_symbol": "DHX32",
  "gene": "UniProtKB:Q7L7V1",
  "term_label": "Unknown biological process",
  "gene_name": "Putative pre-mRNA-splicing factor ATP-dependent RNA helicase DHX32"
}